{
  "gene_symbol": "CD1E",
  "gene": "UniProtKB:P15812",
  "term_id": "GO:0009897",
  "term_label": "external side of plasma membrane",
  "gene_name": "T-cell surface glycoprotein CD1e, membrane-associated"
}